{
  "term_id": "GO:0005886",
  "gene_symbol": "LAT2",
  "gene_name": "Linker for activation of T-cells family member 2",
  "gene": "UniProtKB:Q9GZY6",
  "term_label": "plasma membrane"
}